{
  "term_id": "GO:0005634",
  "term_label": "nucleus",
  "gene_symbol": "TFAP4",
  "gene": "UniProtKB:Q01664",
  "gene_name": "Transcription factor AP-4"
}